{
  "term_label": "Unknown biological process",
  "gene_name": "Myelin expression factor 2",
  "gene_symbol": "MYEF2",
  "term_id": "UNKNOWN:0002",
  "gene": "UniProtKB:Q9P2K5"
}